{
  "term_label": "RNA polymerase II cis-regulatory region sequence-specific DNA binding",
  "gene": "UniProtKB:Q6ISB3",
  "term_id": "GO:0000978",
  "gene_symbol": "GRHL2",
  "gene_name": "Grainyhead-like protein 2 homolog"
}